{
  "gene": "UniProtKB:P98196",
  "term_label": "recycling endosome",
  "gene_symbol": "ATP11A",
  "gene_name": "Phospholipid-transporting ATPase IH",
  "term_id": "GO:0055037"
}